{
  "gene": "UniProtKB:Q9UHD8",
  "gene_name": "Septin-9",
  "term_label": "intracellular protein localization",
  "term_id": "GO:0008104",
  "gene_symbol": "SEPTIN9"
}